cellular response to dsRNA [GO:0071359] (biological process) Definition: Any process that results in a change in state or activity of a cell (in terms of movement, secretion, enzyme production, gene expression, etc.) as a result of a double-stranded RNA stimulus. Subtypes: cellular response to exogenous dsRNA [GO:0071360] Sources: GOC:mah Relationships: is a type of response to dsRNA [GO:0043331]; is a type of cellular response to nitrogen compound [GO:1901699] Also known as: cellular response to double-stranded RNA